{
  "gene_symbol": "NPIPA8",
  "term_label": "Unknown biological process",
  "gene_name": "Nuclear pore complex-interacting protein family member A8",
  "term_id": "UNKNOWN:0002",
  "gene": "UniProtKB:P0DM63"
}